{
  "term_label": "cytosol",
  "gene_symbol": "ALAD",
  "gene_name": "Delta-aminolevulinic acid dehydratase",
  "term_id": "GO:0005829",
  "gene": "UniProtKB:P13716"
}